{
  "term_label": "plasma membrane",
  "gene_name": "Killer cell immunoglobulin-like receptor 2DL2",
  "term_id": "GO:0005886",
  "gene_symbol": "KIR2DL2",
  "gene": "UniProtKB:P43627"
}